{
  "gene": "UniProtKB:Q70CQ3",
  "gene_name": "Ubiquitin carboxyl-terminal hydrolase 30",
  "gene_symbol": "USP30",
  "term_label": "nucleus",
  "term_id": "GO:0005634"
}